{
  "gene_name": "Core-binding factor subunit beta",
  "gene_symbol": "CBFB",
  "gene": "UniProtKB:Q13951",
  "term_label": "regulation of transcription by RNA polymerase II",
  "term_id": "GO:0006357"
}